regulation of aplanospore formation [GO:0075290] (BP) Definition: Any process that modulates the frequency, rate or extent of aplanospore formation, a process in which a nonmotile, asexual spore is formed within a cell in certain algae and fungi (commonly in the Phycomycetes), the wall of aplanospore is distinct from that of the parent cell. Relationships: is a type of regulation of sporangiospore formation [GO:0075286]; regulates aplanospore formation [GO:0075289] Sources: GOC:pamgo_curators Subtypes: positive regulation of aplanospore formation [GO:0075291], GO:0075292